{
  "term_label": "extracellular space",
  "gene_symbol": "SCGB3A1",
  "gene": "UniProtKB:Q96QR1",
  "term_id": "GO:0005615",
  "gene_name": "Secretoglobin family 3A member 1"
}